regulation of antigen processing and presentation of peptide antigen via MHC class Ib [GO:0002595] (biological process) Definition: Any process that modulates the frequency, rate, or extent of antigen processing and presentation of peptide antigen via MHC class Ib. Also known as: regulation of peptide antigen processing and presentation via MHC class Ib Relationships: is a type of GO:0002583; is a type of regulation of antigen processing and presentation via MHC class Ib [GO:0002592]; regulates antigen processing and presentation of peptide antigen via MHC class Ib [GO:0002428] Subtypes: negative regulation of antigen processing and presentation of peptide antigen via MHC class Ib [GO:0002596], positive regulation of antigen processing and presentation of peptide antigen via MHC class Ib [GO:0002597] Sources: GOC:add